{
  "gene_name": "Phosphatidylcholine:ceramide cholinephosphotransferase 2",
  "gene_symbol": "SGMS2",
  "term_label": "Golgi membrane",
  "gene": "UniProtKB:Q8NHU3",
  "term_id": "GO:0000139"
}